{
  "gene_symbol": "MIR1-1HG",
  "term_id": "UNKNOWN:0002",
  "gene": "UniProtKB:Q9H1L0",
  "term_label": "Unknown biological process",
  "gene_name": "Uncharacterized protein MIR1-1HG"
}